{
  "term_label": "transcription coactivator activity",
  "term_id": "GO:0003713",
  "gene_symbol": "SSBP2",
  "gene": "UniProtKB:P81877",
  "gene_name": "Single-stranded DNA-binding protein 2"
}